negative regulation of mesodermal cell fate determination [GO:0048335] (biological process) Relationships: is a type of regulation of mesodermal cell fate determination [GO:0048334]; is a type of negative regulation of cell fate determination [GO:1905934]; negatively regulates GO:0007500 Subtypes: GO:0048325, negative regulation of paraxial mesodermal cell fate determination [GO:0048347], GO:0048375, negative regulation of intermediate mesodermal cell fate determination [GO:0048396] Also known as: down regulation of mesodermal cell fate determination, down-regulation of mesodermal cell fate determination, downregulation of mesodermal cell fate determination, inhibition of mesodermal cell fate determination Sources: GOC:dgh Definition: Any process that stops, prevents, or reduces the frequency, rate or extent of mesoderm cell fate determination.